alpha-beta T cell differentiation [GO:0046632] (biological process) Sources: CL:0000789, GOC:ai Subtypes: NK T cell differentiation [GO:0001865], GO:0002293, GO:0002299, CD4-positive, alpha-beta T cell differentiation [GO:0043367], GO:0043374 Also known as: alpha-beta T lymphocyte differentiation, alpha-beta T-cell differentiation, alpha-beta T-lymphocyte differentiation, alpha-beta T cell development Regulation: regulated by regulation of alpha-beta T cell differentiation [GO:0046637]; positively regulated by positive regulation of alpha-beta T cell differentiation [GO:0046638]; negatively regulated by GO:0046639 Note: Note that immunologists typically use the word 'development' to refer to cells of B or T cell lineages undergoing the process that GO describes as 'cell differentiation'. Relationships: is a type of T cell differentiation [GO:0030217]; is a type of alpha-beta T cell activation [GO:0046631] Definition: The process in which a precursor cell type acquires the specialized features of an alpha-beta T cell. An alpha-beta T cell is a T cell that expresses an alpha-beta T cell receptor complex.